cellular response to interferon-alpha [GO:0035457] (biological process) Also known as: cellular response to leukocyte interferon, cellular response to lymphoblast interferon, cellular response to lymphoblastoid interferon, cellular response to interferon alfa-n1, cellular response to interferon alfa-n3 Relationships: is a type of response to interferon-alpha [GO:0035455]; is_a cellular response to cytokine stimulus [GO:0071345] Definition: Any process that results in a change in state or activity of a cell (in terms of movement, secretion, enzyme production, gene expression, etc.) as a result of an interferon-alpha stimulus. Interferon-alpha is a type I interferon. Sources: GOC:sl